positive regulation of T cell mediated cytotoxicity [GO:0001916] (biological process) Definition: Any process that activates or increases the frequency, rate or extent of T cell mediated cytotoxicity. Subtypes: positive regulation of T cell mediated cytotoxicity directed against tumor cell target [GO:0002854], GO:0043319, susceptibility to T cell mediated cytotoxicity [GO:0060370] Sources: GOC:add, ISBN:0781735149 Relationships: is a type of positive regulation of leukocyte mediated cytotoxicity [GO:0001912]; is a type of regulation of T cell mediated cytotoxicity [GO:0001914]; is a type of positive regulation of T cell mediated immunity [GO:0002711]; positively regulates T cell mediated cytotoxicity [GO:0001913] Also known as: positive regulation of T cell mediated apoptosis, positive regulation of T cell mediated cell death, positive regulation of T cell mediated cell killing, positive regulation of T lymphocyte mediated cytotoxicity, positive regulation of T-cell mediated apoptosis, positive regulation of T-cell mediated cell death, positive regulation of T-cell mediated cell killing, positive regulation of T-cell mediated cytotoxicity, positive regulation of T-lymphocyte mediated cytotoxicity, up regulation of T cell mediated cytotoxicity, up-regulation of T cell mediated cytotoxicity, upregulation of T cell mediated cytotoxicity, activation of T cell mediated cytotoxicity, stimulation of T cell mediated cytotoxicity, positive regulation of T cell mediated cytolysis, positive regulation of T-cell mediated cytolysis